tricarboxylic acid transmembrane transporter activity [GO:0015142] (molecular function) Also known as: sodium:dicarboxylate/tricarboxylate symporter activity Subtypes: citrate transmembrane transporter activity [GO:0015137] Relationships: is_a carboxylic acid transmembrane transporter activity [GO:0046943]; is part of tricarboxylic acid transmembrane transport [GO:0035674] Definition: Enables the transfer of tricarboxylic acids from one side of a membrane to the other. Tricarboxylic acid are organic acids with three COOH groups. Sources: GOC:ai